{
  "gene_name": "Phosphatidylinositol 4,5-bisphosphate 3-kinase catalytic subunit delta isoform",
  "term_label": "cytoplasm",
  "gene": "UniProtKB:O00329",
  "term_id": "GO:0005737",
  "gene_symbol": "PIK3CD"
}